{
  "gene": "UniProtKB:A6NM03",
  "term_label": "detection of chemical stimulus involved in sensory perception of smell",
  "term_id": "GO:0050911",
  "gene_symbol": "OR2AG2",
  "gene_name": "Olfactory receptor 2AG2"
}